{
  "term_label": "respiratory chain complex II (succinate dehydrogenase)",
  "gene_name": "Succinate dehydrogenase [ubiquinone] flavoprotein subunit, mitochondrial",
  "gene_symbol": "SDHA",
  "gene": "UniProtKB:P31040",
  "term_id": "GO:0045273"
}